{
  "gene_symbol": "BRI3BP",
  "term_label": "mitochondrion",
  "gene_name": "BRI3-binding protein",
  "term_id": "GO:0005739",
  "gene": "UniProtKB:Q8WY22"
}